{
  "term_label": "microtubule motor activity",
  "gene_name": "Kinesin-like protein KIF27",
  "term_id": "GO:0003777",
  "gene_symbol": "KIF27",
  "gene": "UniProtKB:Q86VH2"
}